hydrolase activity, acting on carbon-nitrogen (but not peptide) bonds, in linear amidines [GO:0016813] (molecular function) Subtypes: GO:0004037, arginase activity [GO:0004053], protein-arginine deiminase activity [GO:0004668], agmatinase activity [GO:0008783], N-succinylarginine dihydrolase activity [GO:0009015], dimethylargininase activity [GO:0016403], creatinase activity [GO:0016980], arginine deiminase activity [GO:0016990], ammelide aminohydrolase activity [GO:0018754], 2-chloro-4-hydroxy-6-amino-1,3,5-triazine aminohydrolase activity [GO:0018755], ammeline aminohydrolase activity [GO:0018756], deisopropylhydroxyatrazine aminohydrolase activity [GO:0018757], proclavaminate amidinohydrolase activity [GO:0033972], GO:0043730, aminopropylagmatine ureohydrolase activity [GO:0043920], methylenediurea deaminase activity [GO:0047424], GO:0047632, GO:0047652, amidinoaspartase activity [GO:0047660], GO:0047817, diguanidinobutanase activity [GO:0047854], guanidinoacetase activity [GO:0047970], guanidinobutyrase activity [GO:0047971], guanidinopropionase activity [GO:0047972], GO:0050098, formimidoylaspartate deiminase activity [GO:0050414], formimidoylglutamase activity [GO:0050415], formimidoylglutamate deiminase activity [GO:0050416], GO:0071522 Sources: EC:3.5.3.- Relationships: is a type of hydrolase activity, acting on carbon-nitrogen (but not peptide) bonds [GO:0016810] Definition: Catalysis of the hydrolysis of any non-peptide carbon-nitrogen bond in a linear amidine, a compound of the form R-C(=NH)-NH2.